angiostatin binding [GO:0043532] (molecular function) Relationships: is a type of protein binding [GO:0005515] References: PMID:16043488 Definition: Binding to angiostatin, a proteolytic product of plasminogen or plasmin containing at least one intact kringle domain, and which is an inhibitor of angiogenesis.